nuclear lumen [GO:0031981] (cellular component) Definition: The volume enclosed by the nuclear inner membrane. Sources: GOC:mah, GOC:pz Relationships: is a type of intracellular organelle lumen [GO:0070013]; is part of nucleus [GO:0005634]